{
  "term_id": "GO:0061564",
  "gene_symbol": "NEUROD2",
  "gene": "UniProtKB:Q15784",
  "gene_name": "Neurogenic differentiation factor 2",
  "term_label": "axon development"
}